{
  "gene_name": "Ankyrin repeat and SAM domain-containing protein 4B",
  "gene": "UniProtKB:Q8N8V4",
  "gene_symbol": "ANKS4B",
  "term_id": "GO:1904970",
  "term_label": "brush border assembly"
}